{
  "term_id": "GO:0006357",
  "term_label": "regulation of transcription by RNA polymerase II",
  "gene_name": "Zinc finger protein 62 homolog",
  "gene_symbol": "ZFP62",
  "gene": "UniProtKB:Q8NB50"
}